{
  "gene": "UniProtKB:P21860",
  "term_label": "basal plasma membrane",
  "gene_name": "Receptor tyrosine-protein kinase erbB-3",
  "gene_symbol": "ERBB3",
  "term_id": "GO:0009925"
}